fibroblast growth factor receptor binding [GO:0005104] (MF) Subtypes: type 1 fibroblast growth factor receptor binding [GO:0005105], type 2 fibroblast growth factor receptor binding [GO:0005111], GO:0030353 Definition: Binding to a fibroblast growth factor receptor (FGFR). Sources: GOC:ceb Note: Note that branchless is the Drosophila gene encoding fibroblast growth factor. Also known as: fibroblast growth factor, FGF receptor binding, FGFR binding, FGFR ligand, fibroblast growth factor receptor ligand Relationships: is a type of growth factor receptor binding [GO:0070851]